{
  "term_id": "GO:0005654",
  "term_label": "nucleoplasm",
  "gene_symbol": "ARID1B",
  "gene_name": "AT-rich interactive domain-containing protein 1B",
  "gene": "UniProtKB:Q8NFD5"
}